secondary active monocarboxylate transmembrane transporter activity [GO:0015355] (molecular function) Subtypes: GO:0005477, phosphoenolpyruvate:phosphate antiporter activity [GO:0015121], gamma-aminobutyric acid:proton symporter activity [GO:0015495], shikimate:proton symporter activity [GO:0015533], phenyl propionate uniporter activity [GO:0015544], GO:0015649, lactate:proton symporter activity [GO:0015650], GO:0043893, GO:0070909, GO:0140161, gamma-aminobutyric acid:proton antiporter activity [GO:0140800], orotate:monoatomic anion antiporter activity [GO:0140812] Also known as: monocarboxylate porter activity Sources: GOC:bf, GOC:jl Definition: Catalysis of the movement of a monocarboxylate, any compound containing a single carboxyl group (COOH or COO-), by uniport, symport or antiport across a membrane by a carrier-mediated mechanism. Relationships: is a type of monocarboxylic acid transmembrane transporter activity [GO:0008028]; is a type of GO:0015291